{
  "gene_symbol": "CCNB3",
  "term_label": "G1/S transition of mitotic cell cycle",
  "gene": "UniProtKB:Q8WWL7",
  "term_id": "GO:0000082",
  "gene_name": "G2_mitotic-specific cyclin-B3"
}